{
  "term_label": "sulfotransferase activity",
  "gene": "UniProtKB:O00204",
  "term_id": "GO:0008146",
  "gene_symbol": "SULT2B1",
  "gene_name": "Sulfotransferase 2B1"
}